ITP biosynthetic process [GO:0046042] (BP) Definition: The chemical reactions and pathways resulting in the formation of ITP, inosine triphosphate. Relationships: is a type of purine ribonucleotide biosynthetic process [GO:0009152]; is a type of purine ribonucleoside triphosphate biosynthetic process [GO:0009206]; is a type of ITP metabolic process [GO:0046041] Sources: GOC:go_curators Also known as: ITP anabolism, ITP biosynthesis, ITP formation, ITP synthesis